{
  "term_label": "CENP-A containing nucleosome",
  "term_id": "GO:0043505",
  "gene_name": "Histone H3-7",
  "gene": "UniProtKB:Q5TEC6",
  "gene_symbol": "H3-7"
}